{
  "gene": "UniProtKB:P05090",
  "term_id": "GO:0015485",
  "term_label": "cholesterol binding",
  "gene_symbol": "APOD",
  "gene_name": "Apolipoprotein D"
}